{
  "gene_name": "cTAGE family member 9",
  "term_label": "vesicle cargo loading",
  "term_id": "GO:0035459",
  "gene_symbol": "CTAGE9",
  "gene": "UniProtKB:A4FU28"
}